{
  "gene": "UniProtKB:Q9BU02",
  "gene_symbol": "THTPA",
  "term_id": "GO:0000287",
  "term_label": "magnesium ion binding",
  "gene_name": "Thiamine-triphosphatase"
}